regulation of single strand break repair [GO:1903516] (biological process) Relationships: is a type of GO:0006282; regulates single strand break repair [GO:0000012] Definition: Any process that modulates the frequency, rate or extent of single strand break repair. Subtypes: regulation of single-strand break repair via homologous recombination [GO:1903110], negative regulation of single strand break repair [GO:1903517], positive regulation of single strand break repair [GO:1903518] References: PMID:17395247 Sources: GOC:BHF, GOC:TermGenie, GOC:rl, GO_REF:0000058